{
  "gene_symbol": "PKMYT1",
  "gene": "UniProtKB:Q99640",
  "gene_name": "Membrane-associated tyrosine- and threonine-specific cdc2-inhibitory kinase",
  "term_label": "cytoplasm",
  "term_id": "GO:0005737"
}